vascular endothelial cell proliferation [GO:0101023] (biological process) References: PMID:23201774 Sources: GOC:BHF, GOC:BHF_telomere, GOC:nc Definition: The multiplication or reproduction of blood vessel endothelial cells, resulting in the expansion of a cell population. Relationships: is a type of endothelial cell proliferation [GO:0001935] Regulation: regulated by GO:1905562; RO_0002212 by negative regulation of vascular endothelial cell proliferation [GO:1905563]; positively regulated by positive regulation of vascular endothelial cell proliferation [GO:1905564]